{
  "gene": "UniProtKB:P46940",
  "term_id": "GO:0005938",
  "term_label": "cell cortex",
  "gene_name": "Ras GTPase-activating-like protein IQGAP1",
  "gene_symbol": "IQGAP1"
}